{
  "gene_symbol": "CTSZ",
  "gene_name": "Cathepsin Z",
  "term_label": "extracellular space",
  "gene": "UniProtKB:Q9UBR2",
  "term_id": "GO:0005615"
}